aerobic glycerol catabolic process [GO:0019564] (biological process) Relationships: is a type of glycerol catabolic process [GO:0019563] Sources: GOC:ai, ISBN:0198506732 Definition: The chemical reactions and pathways resulting in the breakdown of glycerol, 1,2,3-propanetriol, in the presence of oxygen. Also known as: aerobic glycerol breakdown, aerobic glycerol catabolism, aerobic glycerol degradation, aerobic glycerol fermentation